{
  "gene_symbol": "MUTYH",
  "gene_name": "Adenine DNA glycosylase",
  "term_label": "mismatch repair",
  "gene": "UniProtKB:Q9UIF7",
  "term_id": "GO:0006298"
}